{
  "term_label": "Unknown biological process",
  "gene_name": "Inhibitor of nuclear factor kappa-B kinase-interacting protein",
  "term_id": "UNKNOWN:0002",
  "gene": "UniProtKB:Q70UQ0",
  "gene_symbol": "IKBIP"
}